{
  "gene_symbol": "CEP63",
  "term_label": "centriole",
  "gene": "UniProtKB:Q96MT8",
  "term_id": "GO:0005814",
  "gene_name": "Centrosomal protein of 63 kDa"
}